{
  "term_id": "GO:0005886",
  "gene": "UniProtKB:Q9BY71",
  "term_label": "plasma membrane",
  "gene_symbol": "LRRC3",
  "gene_name": "Leucine-rich repeat-containing protein 3"
}